{
  "term_id": "GO:0007423",
  "gene_name": "Class A basic helix-loop-helix protein 15",
  "gene": "UniProtKB:Q7RTS1",
  "gene_symbol": "BHLHA15",
  "term_label": "sensory organ development"
}